{
  "term_label": "acrosomal vesicle",
  "gene_symbol": "FAM170B",
  "gene_name": "Protein FAM170B",
  "gene": "UniProtKB:A6NMN3",
  "term_id": "GO:0001669"
}